{
  "term_label": "tRNA N1-guanine methylation",
  "gene": "UniProtKB:Q32P41",
  "gene_name": "tRNA (guanine(37)-N1)-methyltransferase",
  "term_id": "GO:0002939",
  "gene_symbol": "TRMT5"
}